{
  "gene_symbol": "KIF23",
  "gene": "UniProtKB:Q02241",
  "term_label": "microtubule binding",
  "gene_name": "Kinesin-like protein KIF23",
  "term_id": "GO:0008017"
}